{
  "gene": "UniProtKB:A0A0A0MT99",
  "gene_symbol": "IGLJ3",
  "term_label": "Unknown cellular component",
  "term_id": "UNKNOWN:0003",
  "gene_name": "Immunoglobulin lambda joining 3 (Fragment)"
}